{
  "gene_symbol": "LPIN3",
  "gene_name": "Phosphatidate phosphatase LPIN3",
  "gene": "UniProtKB:Q9BQK8",
  "term_id": "GO:0003713",
  "term_label": "transcription coactivator activity"
}